{
  "gene_name": "Unconventional myosin-Va",
  "gene": "UniProtKB:Q9Y4I1",
  "gene_symbol": "MYO5A",
  "term_id": "GO:0006897",
  "term_label": "endocytosis"
}